{
  "term_id": "UNKNOWN:0001",
  "gene_name": "T cell receptor alpha joining 41 (Fragment)",
  "gene_symbol": "TRAJ41",
  "gene": "UniProtKB:A0A075B702",
  "term_label": "Unknown molecular function"
}